enniatin biosynthetic process [GO:0046585] (biological process) Definition: The chemical reactions and pathways resulting in the formation of enniatins, any of various cyclodepsipeptide antibiotics from Fusarium species that function as ionophores. Relationships: is a type of antibiotic biosynthetic process [GO:0017000]; is a type of depsipeptide biosynthetic process [GO:0050763]; is_a lactam biosynthetic process [GO:0072339]; is a type of lactone biosynthetic process [GO:1901336] Sources: ISBN:0198506732 Also known as: enniatin anabolism, enniatin biosynthesis, enniatin formation, enniatin synthesis